{
  "term_id": "GO:0005667",
  "gene_symbol": "NFATC3",
  "term_label": "transcription regulator complex",
  "gene": "UniProtKB:Q12968",
  "gene_name": "Nuclear factor of activated T-cells, cytoplasmic 3"
}